positive regulation of B cell chemotaxis [GO:2000538] (biological process) Definition: Any process that activates or increases the frequency, rate or extent of B cell chemotaxis. Relationships: is a type of positive regulation of lymphocyte chemotaxis [GO:0140131]; is_a regulation of B cell chemotaxis [GO:2000537]; positively regulates B cell chemotaxis [GO:0035754] Sources: GOC:obol